{
  "gene": "UniProtKB:Q8NH41",
  "gene_name": "Olfactory receptor 4K15",
  "gene_symbol": "OR4K15",
  "term_label": "olfactory receptor activity",
  "term_id": "GO:0004984"
}